{
  "term_label": "Unknown cellular component",
  "term_id": "UNKNOWN:0003",
  "gene": "UniProtKB:Q6ZUG5",
  "gene_symbol": "Q6ZUG5",
  "gene_name": "Uncharacterized protein FLJ43738"
}